{
  "gene_name": "Protein APCDD1",
  "term_id": "GO:0017147",
  "gene": "UniProtKB:Q8J025",
  "gene_symbol": "APCDD1",
  "term_label": "Wnt-protein binding"
}